{
  "gene_symbol": "VSIG2",
  "gene_name": "V-set and immunoglobulin domain-containing protein 2",
  "term_id": "UNKNOWN:0001",
  "term_label": "Unknown molecular function",
  "gene": "UniProtKB:Q96IQ7"
}